{
  "gene_symbol": "SPATA12",
  "gene_name": "Spermatogenesis-associated protein 12",
  "gene": "UniProtKB:Q7Z6I5",
  "term_id": "UNKNOWN:0001",
  "term_label": "Unknown molecular function"
}